blood vessel endothelial cell migration involved in intussusceptive angiogenesis [GO:0002044] (biological process) References: PMID:16391003 Definition: The orderly movement of endothelial cells into the extracellular matrix in order to form new blood vessels during intussusceptive angiogenesis. Relationships: is a type of blood vessel endothelial cell migration [GO:0043534]; is part of intussusceptive angiogenesis [GO:0002041]